mitochondrial tRNA pseudouridine synthesis [GO:0070902] (biological process) Relationships: is a type of GO:0031119; is a type of mitochondrial tRNA modification [GO:0070900] Sources: GOC:mah, GOC:mcc Definition: The intramolecular conversion of uridine to pseudouridine in a mitochondrial tRNA molecule.